{
  "term_id": "UNKNOWN:0003",
  "gene_name": "Putative uncharacterized protein encoded by LINC00575",
  "gene": "UniProtKB:Q6W349",
  "gene_symbol": "LINC00575",
  "term_label": "Unknown cellular component"
}